{
  "term_label": "heart morphogenesis",
  "gene_symbol": "MESP2",
  "term_id": "GO:0003007",
  "gene": "UniProtKB:Q0VG99",
  "gene_name": "Mesoderm posterior protein 2"
}